{
  "term_label": "inflammatory response",
  "gene_symbol": "TAC4",
  "gene": "UniProtKB:Q86UU9",
  "term_id": "GO:0006954",
  "gene_name": "Tachykinin-4"
}